{
  "gene_symbol": "SLCO3A1",
  "term_label": "prostaglandin transport",
  "gene_name": "Solute carrier organic anion transporter family member 3A1",
  "gene": "UniProtKB:Q9UIG8",
  "term_id": "GO:0015732"
}